{
  "term_label": "kainate selective glutamate receptor complex",
  "gene_symbol": "GRIK1",
  "term_id": "GO:0032983",
  "gene_name": "Glutamate receptor ionotropic, kainate 1",
  "gene": "UniProtKB:P39086"
}